acidic amino acid transport [GO:0015800] (biological process) Subtypes: GO:0014047, aspartate transmembrane transport [GO:0015810], L-glutamate import [GO:0051938], gamma-aminobutyric acid import [GO:0051939], aspartate secretion [GO:0061528], glutamate transmembrane import into vacuole [GO:0090454] Relationships: is a type of amino acid transport [GO:0006865] Definition: The directed movement of acidic amino acids, amino acids with a pH below 7, into, out of or within a cell, or between cells, by means of some agent such as a transporter or pore. Sources: GOC:ai